{
  "gene_name": "C-type lectin domain family 6 member A",
  "gene": "UniProtKB:Q6EIG7",
  "term_id": "GO:0061760",
  "term_label": "antifungal innate immune response",
  "gene_symbol": "CLEC6A"
}